{
  "gene_symbol": "FLG",
  "gene_name": "Filaggrin",
  "gene": "UniProtKB:P20930",
  "term_label": "cornified envelope",
  "term_id": "GO:0001533"
}